{
  "term_label": "guanyl-nucleotide exchange factor activity",
  "gene": "UniProtKB:Q96PE2",
  "gene_name": "Rho guanine nucleotide exchange factor 17",
  "gene_symbol": "ARHGEF17",
  "term_id": "GO:0005085"
}